{
  "gene_name": "Peptidylprolyl isomerase domain and WD repeat-containing protein 1",
  "term_id": "GO:0003755",
  "gene": "UniProtKB:Q96BP3",
  "term_label": "peptidyl-prolyl cis-trans isomerase activity",
  "gene_symbol": "PPWD1"
}